{
  "gene_symbol": "AQR",
  "gene": "UniProtKB:O60306",
  "term_id": "GO:0071013",
  "term_label": "catalytic step 2 spliceosome",
  "gene_name": "RNA helicase aquarius"
}